{
  "term_id": "UNKNOWN:0001",
  "gene_symbol": "ZFYVE27",
  "term_label": "Unknown molecular function",
  "gene_name": "Protrudin",
  "gene": "UniProtKB:Q5T4F4"
}